{
  "gene_name": "Thy-1 membrane glycoprotein",
  "term_label": "positive regulation of focal adhesion assembly",
  "gene_symbol": "THY1",
  "term_id": "GO:0051894",
  "gene": "UniProtKB:P04216"
}